riboflavin kinase activity [GO:0008531] (molecular function) Sources: EC:2.7.1.26, RHEA:14357 Definition: Catalysis of the reaction: ATP + riboflavin = ADP + FMN + 2 H+. Also known as: ATP:riboflavin 5'-phosphotransferase activity, FK, flavokinase activity, riboflavin kinase (phosphorylating), riboflavine kinase activity Relationships: is a type of kinase activity [GO:0016301]; is a type of phosphotransferase activity, alcohol group as acceptor [GO:0016773]